{
  "gene_name": "Astrocytic phosphoprotein PEA-15",
  "term_id": "UNKNOWN:0003",
  "term_label": "Unknown cellular component",
  "gene_symbol": "PEA15",
  "gene": "UniProtKB:Q15121"
}